{
  "term_id": "GO:0043022",
  "gene_name": "Small ribosomal subunit protein RACK1",
  "term_label": "ribosome binding",
  "gene": "UniProtKB:P63244",
  "gene_symbol": "RACK1"
}